{
  "gene_symbol": "WDR43",
  "term_label": "maturation of SSU-rRNA from tricistronic rRNA transcript (SSU-rRNA, 5.8S rRNA, LSU-rRNA)",
  "gene_name": "WD repeat-containing protein 43",
  "gene": "UniProtKB:Q15061",
  "term_id": "GO:0000462"
}